{
  "term_label": "3',5'-cyclic-AMP phosphodiesterase activity",
  "gene_symbol": "PDE6B",
  "gene": "UniProtKB:P35913",
  "term_id": "GO:0004115",
  "gene_name": "Rod cGMP-specific 3',5'-cyclic phosphodiesterase subunit beta"
}